regulation of toll-like receptor 4 signaling pathway [GO:0034143] (biological process) Definition: Any process that modulates the frequency, rate, or extent of toll-like receptor 4 signaling pathway. References: PMID:16551253, PMID:17328678 Sources: GOC:add Relationships: is a type of GO:0062207; regulates GO:0034142 Subtypes: negative regulation of toll-like receptor 4 signaling pathway [GO:0034144], positive regulation of toll-like receptor 4 signaling pathway [GO:0034145] Also known as: regulation of TLR4 signaling pathway, regulation of toll-like receptor 4 signalling pathway